{
  "gene_name": "Sperm equatorial segment protein 1",
  "gene_symbol": "SPESP1",
  "gene": "UniProtKB:Q6UW49",
  "term_label": "acrosomal vesicle",
  "term_id": "GO:0001669"
}